{
  "term_id": "GO:0005615",
  "term_label": "extracellular space",
  "gene_name": "Protein Z-dependent protease inhibitor",
  "gene_symbol": "SERPINA10",
  "gene": "UniProtKB:Q9UK55"
}